negative regulation of chromosome condensation [GO:1902340] (biological process) Subtypes: negative regulation of mitotic chromosome condensation [GO:1905213] References: PMID:23219725 Sources: GOC:TermGenie Also known as: down regulation of chromosome condensation, down regulation of eukaryotic chromosome condensation, down regulation of nuclear chromosome condensation, down-regulation of chromosome condensation, down-regulation of eukaryotic chromosome condensation, down-regulation of nuclear chromosome condensation, downregulation of chromosome condensation, downregulation of eukaryotic chromosome condensation, downregulation of nuclear chromosome condensation, negative regulation of eukaryotic chromosome condensation, negative regulation of nuclear chromosome condensation, inhibition of chromosome condensation, inhibition of eukaryotic chromosome condensation, inhibition of nuclear chromosome condensation Relationships: is a type of regulation of chromosome condensation [GO:0060623]; is_a negative regulation of chromosome organization [GO:2001251]; negatively regulates chromosome condensation [GO:0030261] Definition: Any process that stops, prevents or reduces the frequency, rate or extent of chromosome condensation.